{
  "term_id": "GO:0042056",
  "gene_name": "Placenta growth factor",
  "gene_symbol": "PGF",
  "gene": "UniProtKB:P49763",
  "term_label": "chemoattractant activity"
}